{
  "gene": "UniProtKB:Q0P641",
  "term_label": "Unknown cellular component",
  "term_id": "UNKNOWN:0003",
  "gene_name": "Uncharacterized protein C2orf80",
  "gene_symbol": "C2orf80"
}